{
  "gene_name": "Prostaglandin G_H synthase 2",
  "gene": "UniProtKB:P35354",
  "term_id": "GO:0019371",
  "gene_symbol": "PTGS2",
  "term_label": "cyclooxygenase pathway"
}